somatotropin secreting cell development [GO:0060133] (BP) Sources: GOC:dph Definition: The process whose specific outcome is the progression of a somatotropin secreting cell over time, from its formation to the mature structure. A somatotropin secreting cell is an acidophilic cell of the anterior pituitary that produces growth hormone, somatotropin. Relationships: is a type of cell development [GO:0048468]; BFO_0000050 GO:0060126 Also known as: growth hormone secreting cell development, somatotrophin secreting cell development, somatotropic cell development, somatotrope development, somatotroph development, somatrophic cell development